{
  "term_label": "phagophore",
  "gene": "UniProtKB:Q96BY7",
  "gene_symbol": "ATG2B",
  "gene_name": "Autophagy-related protein 2 homolog B",
  "term_id": "GO:0061908"
}